{
  "gene_symbol": "XIRP1",
  "gene_name": "Xin actin-binding repeat-containing protein 1",
  "term_id": "GO:0001725",
  "gene": "UniProtKB:Q702N8",
  "term_label": "stress fiber"
}